{
  "gene_name": "Paraneoplastic antigen-like protein 8A",
  "gene_symbol": "PNMA8A",
  "term_id": "UNKNOWN:0002",
  "term_label": "Unknown biological process",
  "gene": "UniProtKB:Q86V59"
}